{
  "gene_name": "Syntaphilin",
  "term_label": "Unknown molecular function",
  "gene_symbol": "SNPH",
  "term_id": "UNKNOWN:0001",
  "gene": "UniProtKB:O15079"
}